phosphatidylinositol-3,4-bisphosphate 4-phosphatase activity [GO:0016316] (molecular function) Sources: GOC:hb, RHEA:17193 Definition: Catalysis of the reaction: 1-phosphatidyl-1D-myo-inositol 3,4-bisphosphate + H2O = 1-phosphatidyl-1D-myo-inositol 3-phosphate + phosphate. Also known as: 1-phosphatidyl-1D-myo-inositol-3,4-bisphosphate 4-phosphohydrolase activity, inositol polyphosphate 4-phosphatase type II activity Relationships: is a type of GO:0034596; is a type of GO:0106017; is part of phosphatidylinositol-3-phosphate biosynthetic process [GO:0036092]